regulation of nucleotide-excision repair [GO:2000819] (BP) Relationships: is a type of GO:0006282; regulates nucleotide-excision repair [GO:0006289] Definition: Any process that modulates the frequency, rate or extent of nucleotide-excision repair. Subtypes: regulation of transcription-coupled nucleotide-excision repair [GO:0090262] References: PMID:18836076 Sources: GOC:jp Also known as: regulation of NER, regulation of pyrimidine-dimer repair, DNA damage excision, regulation of interstrand crosslink repair, regulation of intrastrand cross-link repair